{
  "term_label": "interleukin-17 receptor activity",
  "gene": "UniProtKB:Q6ZVW7",
  "term_id": "GO:0030368",
  "gene_name": "Putative interleukin-17 receptor E-like",
  "gene_symbol": "IL17REL"
}